{
  "gene": "UniProtKB:Q9UM01",
  "gene_symbol": "SLC7A7",
  "term_id": "GO:0003333",
  "gene_name": "Y+L amino acid transporter 1",
  "term_label": "amino acid transmembrane transport"
}